{
  "term_id": "GO:0007198",
  "gene": "UniProtKB:P28221",
  "term_label": "adenylate cyclase-inhibiting serotonin receptor signaling pathway",
  "gene_name": "5-hydroxytryptamine receptor 1D",
  "gene_symbol": "HTR1D"
}